{
  "gene_symbol": "FAM110D",
  "term_label": "Unknown molecular function",
  "term_id": "UNKNOWN:0001",
  "gene": "UniProtKB:Q8TAY7",
  "gene_name": "Protein FAM110D"
}